{
  "gene": "UniProtKB:P02749",
  "term_id": "UNKNOWN:0003",
  "gene_name": "Beta-2-glycoprotein 1",
  "term_label": "Unknown cellular component",
  "gene_symbol": "APOH"
}